negative regulation of plant-type cell wall cellulose catabolic process [GO:2000940] (biological process) Also known as: negative regulation of plant-type cell wall polysaccharide breakdown Relationships: is a type of GO:2000939; is a type of negative regulation of cell wall polysaccharide catabolic process [GO:2000967]; negatively regulates plant-type cell wall cellulose catabolic process [GO:0044348] Definition: Any process that stops, prevents or reduces the frequency, rate or extent of plant-type cell wall cellulose catabolic process. Sources: GOC:mengo_curators